{
  "gene": "UniProtKB:P85298",
  "gene_symbol": "ARHGAP8",
  "term_id": "GO:0007264",
  "term_label": "small GTPase-mediated signal transduction",
  "gene_name": "Rho GTPase-activating protein 8"
}